{
  "gene_name": "Vimentin",
  "gene_symbol": "VIM",
  "gene": "UniProtKB:P08670",
  "term_label": "structural constituent of cytoskeleton",
  "term_id": "GO:0005200"
}